{
  "gene_name": "Rho-related GTP-binding protein RhoV",
  "term_id": "GO:0005525",
  "gene": "UniProtKB:Q96L33",
  "term_label": "GTP binding",
  "gene_symbol": "RHOV"
}